{
  "term_label": "Unknown biological process",
  "gene_name": "Cilia- and flagella-associated protein 46",
  "term_id": "UNKNOWN:0002",
  "gene": "UniProtKB:Q8IYW2",
  "gene_symbol": "CFAP46"
}